{
  "gene_symbol": "HOXD4",
  "gene_name": "Homeobox protein Hox-D4",
  "term_id": "GO:0009952",
  "term_label": "anterior/posterior pattern specification",
  "gene": "UniProtKB:P09016"
}